{
  "gene_name": "Serine_threonine-protein phosphatase 4 regulatory subunit 2",
  "gene": "UniProtKB:Q9NY27",
  "term_id": "GO:0030289",
  "gene_symbol": "PPP4R2",
  "term_label": "protein phosphatase 4 complex"
}